alpha-tubulin binding [GO:0043014] (molecular function) Definition: Binding to the microtubule constituent protein alpha-tubulin. Sources: GOC:jl Relationships: is a type of tubulin binding [GO:0015631] Also known as: alpha tubulin binding